{
  "gene": "UniProtKB:P13498",
  "term_label": "superoxide anion generation",
  "gene_symbol": "CYBA",
  "term_id": "GO:0042554",
  "gene_name": "Cytochrome b-245 light chain"
}